suberin network [GO:0048225] (cellular component) Definition: An extracellular matrix part that consists of fatty acid-derived polymers, including both aromatic and aliphatic components. The suberin network is found in specialized plant cell walls, where it is laid down between the primary wall and plasma membrane, forms protective and wound-healing layers, and provides a water-impermeable diffusion barrier. Relationships: is a type of GO:0110165; is part of secondary cell wall [GO:0009531] References: PMID:18440267, PMID:7706282 Sources: GOC:jid, GOC:mah